{
  "gene_name": "Interleukin-10",
  "gene_symbol": "IL10",
  "gene": "UniProtKB:P22301",
  "term_id": "GO:0006955",
  "term_label": "immune response"
}